{
  "term_id": "UNKNOWN:0002",
  "gene": "UniProtKB:Q6ZNB5",
  "term_label": "Unknown biological process",
  "gene_symbol": "XNDC1N",
  "gene_name": "Protein XNDC1N"
}